{
  "term_label": "chaperonin-containing T-complex",
  "term_id": "GO:0005832",
  "gene": "UniProtKB:Q99832",
  "gene_symbol": "CCT7",
  "gene_name": "T-complex protein 1 subunit eta"
}